{
  "gene": "UniProtKB:Q8TDI0",
  "term_label": "nucleus",
  "term_id": "GO:0005634",
  "gene_symbol": "CHD5",
  "gene_name": "Chromodomain-helicase-DNA-binding protein 5"
}